negative regulation of Wnt signaling pathway [GO:0030178] (biological process) Relationships: is a type of negative regulation of signal transduction [GO:0009968]; is a type of regulation of Wnt signaling pathway [GO:0030111]; negatively regulates Wnt signaling pathway [GO:0016055] Also known as: down regulation of Wnt receptor signaling pathway, down regulation of frizzled signaling pathway, down-regulation of Wnt receptor signaling pathway, down-regulation of frizzled signaling pathway, downregulation of Wnt receptor signaling pathway, downregulation of frizzled signaling pathway, negative regulation of Wnt receptor signaling pathway, negative regulation of Wnt receptor signalling pathway, negative regulation of Wnt-activated signaling pathway, negative regulation of frizzled signaling pathway, negative regulation of frizzled signalling pathway, inhibition of Wnt receptor signaling pathway, inhibition of frizzled signaling pathway Subtypes: GO:0003308, negative regulation of canonical Wnt signaling pathway [GO:0090090], negative regulation of non-canonical Wnt signaling pathway [GO:2000051] Definition: Any process that stops, prevents, or reduces the frequency, rate or extent of the Wnt signaling pathway. Sources: GOC:dph, GOC:go_curators, GOC:tb